{
  "term_id": "GO:0006357",
  "gene_name": "Homeobox protein Hox-B9",
  "gene_symbol": "HOXB9",
  "term_label": "regulation of transcription by RNA polymerase II",
  "gene": "UniProtKB:P17482"
}